{
  "term_label": "nucleus",
  "gene_name": "T-box transcription factor T",
  "gene": "UniProtKB:O15178",
  "term_id": "GO:0005634",
  "gene_symbol": "TBXT"
}